methyl-CpNpN binding [GO:0010429] (molecular function) Relationships: is a type of nucleotide binding [GO:0000166] Definition: Binding to a methylated cytosine/unspecified/unspecified trinucleotide. References: PMID:17239600